{
  "gene_symbol": "GRB10",
  "gene_name": "Growth factor receptor-bound protein 10",
  "term_id": "GO:0008286",
  "term_label": "insulin receptor signaling pathway",
  "gene": "UniProtKB:Q13322"
}